{
  "term_id": "GO:0035556",
  "gene": "UniProtKB:P23743",
  "gene_symbol": "DGKA",
  "term_label": "intracellular signal transduction",
  "gene_name": "Diacylglycerol kinase alpha"
}